L-glutamate transmembrane transporter activity [GO:0005313] (molecular function) Sources: GOC:ai, GOC:mtg_transport, ISBN:0815340729 Subtypes: high-affinity L-glutamate transmembrane transporter activity [GO:0005314], cystine:glutamate antiporter activity [GO:0015327], GO:0106421, L-glutamate uniporter activity [GO:0140788] Definition: Enables the transfer of L-glutamate from one side of a membrane to the other. L-glutamate is the anion of 2-aminopentanedioic acid. Also known as: L-glutamate transporter activity, glutamate transmembrane transporter activity, glutamate/aspartate porter activity, glutamate/aspartate:sodium symporter activity Relationships: is a type of acidic amino acid transmembrane transporter activity [GO:0015172]; is_a GO:0015179; is part of L-glutamate transmembrane transport [GO:0015813]